{
  "term_id": "GO:0005886",
  "term_label": "plasma membrane",
  "gene_name": "Scavenger receptor cysteine-rich type 1 protein M160",
  "gene": "UniProtKB:Q9NR16",
  "gene_symbol": "CD163L1"
}